nuclear membrane microtubule tethering complex [GO:0106094] (cellular component) Subtypes: meiotic nuclear membrane microtubule tethering complex [GO:0034993], mitotic nuclear membrane microtubule tethering complex [GO:0106084] Definition: A nuclear membrane protein complex which connects the nuclear outer and inner membranes together, and links thereby links the nuclear lumen to cytoplasmic microtubules. References: PMID:19225124 Sources: GOC:vw Relationships: is a type of nuclear membrane protein complex [GO:0106083]